{
  "term_label": "Unknown cellular component",
  "gene": "UniProtKB:Q9Y5Y3",
  "term_id": "UNKNOWN:0003",
  "gene_name": "Probable G-protein coupled receptor 45",
  "gene_symbol": "GPR45"
}